{
  "term_label": "nervous system development",
  "gene_name": "Laminin subunit alpha-4",
  "term_id": "GO:0007399",
  "gene_symbol": "LAMA4",
  "gene": "UniProtKB:Q16363"
}